{
  "term_id": "UNKNOWN:0002",
  "term_label": "Unknown biological process",
  "gene_symbol": "TMX3",
  "gene_name": "Protein disulfide-isomerase TMX3",
  "gene": "UniProtKB:Q96JJ7"
}